negative regulation of aorta morphogenesis [GO:1903848] (biological process) References: PMID:22269326 Sources: GOC:BHF, GOC:BHF_miRNA, GOC:TermGenie, GOC:rph, GO_REF:0000058 Definition: Any process that stops, prevents or reduces the frequency, rate or extent of aorta morphogenesis. Also known as: down regulation of aorta morphogenesis, down-regulation of aorta morphogenesis, downregulation of aorta morphogenesis, inhibition of aorta morphogenesis Relationships: is a type of regulation of aorta morphogenesis [GO:1903847]; is a type of negative regulation of artery morphogenesis [GO:1905652]; negatively regulates aorta morphogenesis [GO:0035909]